negative regulation of polarized epithelial cell differentiation [GO:0030861] (biological process) Sources: GOC:mah Also known as: down regulation of polarized epithelial cell differentiation, down-regulation of polarized epithelial cell differentiation, downregulation of polarized epithelial cell differentiation, inhibition of polarized epithelial cell differentiation Relationships: is a type of negative regulation of epithelial cell differentiation [GO:0030857]; is a type of regulation of polarized epithelial cell differentiation [GO:0030860]; negatively regulates GO:0030859 Definition: Any process that stops, prevents, or reduces the frequency, rate or extent of polarized epithelial cell differentiation.